{
  "gene": "UniProtKB:O94813",
  "term_label": "Unknown cellular component",
  "term_id": "UNKNOWN:0003",
  "gene_symbol": "SLIT2",
  "gene_name": "Slit homolog 2 protein"
}